{
  "gene": "UniProtKB:P52803",
  "term_id": "GO:0048013",
  "gene_symbol": "EFNA5",
  "term_label": "ephrin receptor signaling pathway",
  "gene_name": "Ephrin-A5"
}